{
  "gene": "UniProtKB:Q92928",
  "gene_symbol": "RAB1C",
  "term_label": "endomembrane system",
  "gene_name": "Putative Ras-related protein Rab-1C",
  "term_id": "GO:0012505"
}